{
  "term_id": "UNKNOWN:0001",
  "term_label": "Unknown molecular function",
  "gene": "UniProtKB:Q8N0Z6",
  "gene_symbol": "TTC5",
  "gene_name": "Tetratricopeptide repeat protein 5"
}